{
  "gene": "UniProtKB:Q13608",
  "term_label": "protein import into peroxisome matrix",
  "gene_symbol": "PEX6",
  "gene_name": "Peroxisomal ATPase PEX6",
  "term_id": "GO:0016558"
}